{
  "gene": "UniProtKB:Q8IXZ2",
  "term_id": "UNKNOWN:0002",
  "term_label": "Unknown biological process",
  "gene_name": "Zinc finger CCCH domain-containing protein 3",
  "gene_symbol": "ZC3H3"
}